{
  "gene_symbol": "IGBP1C",
  "term_label": "regulation of dephosphorylation",
  "gene": "UniProtKB:A0A1W2PR95",
  "gene_name": "Immunoglobulin-binding protein 1 family member C",
  "term_id": "GO:0035303"
}